{
  "gene": "UniProtKB:Q6ZTN6",
  "gene_symbol": "ANKRD13D",
  "term_id": "GO:0005886",
  "gene_name": "Ankyrin repeat domain-containing protein 13D",
  "term_label": "plasma membrane"
}